sinoatrial valve morphogenesis [GO:0003185] (biological process) Definition: The process in which the structure of the sinoatrial valve is generated and organized. Sources: GOC:mtg_heart Relationships: is a type of GO:0003179; is part of GO:0003172 Also known as: SA valve morphogenesis